{
  "gene_symbol": "A2M",
  "gene": "UniProtKB:P01023",
  "gene_name": "Alpha-2-macroglobulin",
  "term_id": "GO:0002020",
  "term_label": "protease binding"
}